{
  "term_id": "GO:0005516",
  "term_label": "calmodulin binding",
  "gene": "UniProtKB:Q9H2S1",
  "gene_symbol": "KCNN2",
  "gene_name": "Small conductance calcium-activated potassium channel protein 2"
}